{
  "gene_symbol": "MRPL19",
  "gene": "UniProtKB:P49406",
  "term_label": "Unknown biological process",
  "gene_name": "Large ribosomal subunit protein bL19m",
  "term_id": "UNKNOWN:0002"
}